{
  "term_id": "GO:0045202",
  "gene_name": "Double C2-like domain-containing protein alpha",
  "term_label": "synapse",
  "gene_symbol": "DOC2A",
  "gene": "UniProtKB:Q14183"
}